{
  "term_label": "negative regulation of DNA-templated transcription",
  "gene": "UniProtKB:Q99750",
  "gene_symbol": "MDFI",
  "term_id": "GO:0045892",
  "gene_name": "MyoD family inhibitor"
}